adenine/guanine mispair binding [GO:0035485] (molecular function) Definition: Binding to a double-stranded DNA region containing an A/G mispair. Sources: GOC:bf, GOC:jh Also known as: A/G mispair binding, guanine-adenine mispair binding, G/A mispair binding Relationships: is_a mismatched DNA binding [GO:0030983]